{
  "term_id": "GO:0001517",
  "gene_name": "Carbohydrate sulfotransferase 1",
  "gene": "UniProtKB:O43916",
  "gene_symbol": "CHST1",
  "term_label": "N-acetylglucosamine 6-O-sulfotransferase activity"
}